{
  "gene": "UniProtKB:Q8IYV9",
  "gene_name": "Izumo sperm-egg fusion protein 1",
  "gene_symbol": "IZUMO1",
  "term_label": "receptor ligand activity",
  "term_id": "GO:0048018"
}